unsaturated monocarboxylic acid metabolic process [GO:0032789] (biological process) Also known as: unsaturated monocarboxylate metabolic process, unsaturated monocarboxylic acid metabolism Sources: GOC:mah, GOC:vk Definition: The chemical reactions and pathways involving unsaturated monocarboxylic acids, any organic acid containing one carboxyl (COOH) group or anion (COO-) and one or more unsaturated C-C bonds. Relationships: is_a GO:0032787